{
  "term_label": "regulation of protein stability",
  "gene": "UniProtKB:Q0WX57",
  "term_id": "GO:0031647",
  "gene_name": "Ubiquitin carboxyl-terminal hydrolase 17-like protein 24",
  "gene_symbol": "USP17L30"
}